{
  "term_id": "GO:0016887",
  "term_label": "ATP hydrolysis activity",
  "gene": "UniProtKB:P48723",
  "gene_name": "Heat shock 70 kDa protein 13",
  "gene_symbol": "HSPA13"
}